{
  "gene_name": "Immunity-related GTPase family M protein",
  "gene": "UniProtKB:A1A4Y4",
  "gene_symbol": "IRGM",
  "term_id": "GO:0005789",
  "term_label": "endoplasmic reticulum membrane"
}